{
  "term_id": "UNKNOWN:0001",
  "gene": "UniProtKB:Q96M43",
  "gene_symbol": "NBPF4",
  "gene_name": "Neuroblastoma breakpoint family member 4",
  "term_label": "Unknown molecular function"
}